(R)-2-hydroxyglutarate dehydrogenase activity [GO:0051990] (molecular function) Sources: RHEA:38295 Subtypes: GO:0099615, (R)-2-hydroxyglutarate (NAD+) dehydrogenase activity [GO:0120568] Relationships: is a type of oxidoreductase activity, acting on CH-OH group of donors [GO:0016614] Definition: Catalysis of the reaction: (R)-2-hydroxyglutarate + acceptor = 2-oxoglutarate + reduced acceptor. Also known as: D-2-hydroxyglutarate dehydrogenase activity